adaptive immune effector response involving T cells and B lineage cells [GO:0090719] (biological process) Sources: GOC:add, ISBN:1405196831 Definition: An adaptive immune effector response involving T cells and B lineage cells. In the case of B lineage cells, the effector cells are the antibody secreting plasma cells whereas for T cells the effector cells may be helper T cells or cytotoxic T cells. Relationships: is a type of adaptive immune response based on somatic recombination of immune receptors built from immunoglobulin superfamily domains [GO:0002460]; is_a GO:0090718